clathrin coating of Golgi vesicle [GO:0048202] (biological process) Subtypes: clathrin coating of Golgi vesicle, plasma membrane to endosome targeting [GO:0010785], clathrin coating of Golgi vesicle, trans-Golgi to endosome targeting [GO:0010786] Also known as: clathrin coating of Golgi-derived vesicle References: PMID:10219233 Sources: GOC:jid, GOC:mah, ISBN:0716731363 Definition: The addition of clathrin and adaptor proteins to Golgi membranes during the formation of transport vesicles, forming a vesicle coat. Relationships: is a type of GO:0048200; is a type of GO:0048268